left middle basal body pair [GO:0097563] (cellular component) Definition: Set of two basal bodies found in Giardia species (trophozoite stage). It comprises the caudal and posteriolateral basal bodies located to the right of the left nucleus of the trophozoite when viewed dorsally. Note: Due to the asymmetric nature of the Giardia trophozoite, this term is defined spatially as the trophozoite is viewed from the dorsal side, with the two nuclei dorsal to the ventral disc, and the ventral disc toward the anterior. Relationships: is a type of cellular anatomical structure [GO:0110165]; is part of cell projection [GO:0042995]; has part left posteriolateral basal body [GO:1902673]; has part left caudal basal body [GO:1902677] References: PMID:16607022, PMID:5961344 Sources: GOC:giardia, ISBN:9780124260207